{
  "term_label": "membrane",
  "gene_name": "Long-chain-fatty-acid--CoA ligase 5",
  "gene": "UniProtKB:Q9ULC5",
  "term_id": "GO:0016020",
  "gene_symbol": "ACSL5"
}